{
  "term_label": "Unknown biological process",
  "term_id": "UNKNOWN:0002",
  "gene_name": "Aquaporin-11",
  "gene_symbol": "AQP11",
  "gene": "UniProtKB:Q8NBQ7"
}